protein adenylylation [GO:0018117] (biological process) Subtypes: peptidyl-histidine adenylylation [GO:0051111] Relationships: is a type of protein nucleotidylation [GO:0018175] Regulation: RO_0002211 by regulation of protein adenylylation [GO:1900722]; negatively regulated by GO:1900723; RO_0002213 by GO:1900724 Also known as: protein AMPylation, protein adenylation, protein amino acid adenylylation References: PMID:21607083 Sources: GOC:ai, GOC:jsg, GOC:sart Definition: The addition of an adenylyl group (adenosine 5'-monophosphate; AMP) to a protein amino acid.